baroreceptor response to increased systemic arterial blood pressure [GO:0001983] (biological process) Definition: The increase in nerve impulses from baroreceptors as a result of increased pressure on an artery that results in an inhibition of sympathetic nerve impulses to peripheral blood vessels. Relationships: is a type of regulation of systemic arterial blood pressure by carotid sinus baroreceptor feedback [GO:0001978]; is a type of negative regulation of systemic arterial blood pressure [GO:0003085] Sources: GOC:mtg_cardio, ISBN:0323031951, ISBN:0721643949